{
  "gene_name": "Solute carrier family 25 member 47",
  "term_id": "GO:0005739",
  "gene_symbol": "SLC25A47",
  "gene": "UniProtKB:Q6Q0C1",
  "term_label": "mitochondrion"
}